{
  "gene": "UniProtKB:A0A087X1G2",
  "term_id": "GO:0005096",
  "gene_symbol": "TBC1D3K",
  "term_label": "GTPase activator activity",
  "gene_name": "TBC1 domain family member 3K"
}